{
  "gene": "UniProtKB:P35212",
  "gene_name": "Gap junction alpha-4 protein",
  "term_label": "gap junction channel activity",
  "gene_symbol": "GJA4",
  "term_id": "GO:0005243"
}